nicotinamide phosphoribosyltransferase activity [GO:0047280] (molecular function) Definition: Catalysis of the reaction: diphosphate + nicotinamide mononucleotide = 5-phospho-alpha-D-ribose 1-diphosphate + H+ + nicotinamide. Sources: RHEA:16149 Also known as: NMN diphosphorylase activity, NMN pyrophosphorylase activity, NMN synthetase activity, nicotinamide mononucleotide pyrophosphorylase activity, nicotinamide mononucleotide synthetase activity, nicotinamide-nucleotide:diphosphate phospho-alpha-D-ribosyltransferase activity Relationships: is a type of pentosyltransferase activity [GO:0016763]